kidney mesenchyme development [GO:0072074] (biological process) Definition: The biological process whose specific outcome is the progression of a kidney mesenchyme from an initial condition to its mature state. This process begins with the formation of kidney mesenchyme and ends with the mature structure. Kidney mesenchyme is the tissue made up of loosely connected mesenchymal cells in the kidney. Sources: GOC:mtg_kidney_jan10 Relationships: is_a GO:0060485; is part of kidney development [GO:0001822] Subtypes: mesonephric mesenchyme development [GO:0061219], GO:0072072, metanephric mesenchyme development [GO:0072075], nephrogenic mesenchyme development [GO:0072076]